L-kynurenine metabolic process [GO:0097052] (biological process) Subtypes: L-kynurenine catabolic process [GO:0097053] Also known as: L-kynurenine metabolism Relationships: is a type of kynurenine metabolic process [GO:0070189]; is a type of L-amino acid metabolic process [GO:0170033] Definition: The chemical reactions and pathways involving L-kynurenine, the L-enantiomer of the amino acid kynurenine (3-(2-aminobenzoyl)-alanine). Sources: GOC:yaf